negative regulation of T-helper 2 cell cytokine production [GO:2000552] (BP) Also known as: negative regulation of Th2 cell cytokine production Relationships: is a type of negative regulation of T cell cytokine production [GO:0002725]; is_a GO:0002829; is_a regulation of T-helper 2 cell cytokine production [GO:2000551]; negatively regulates T-helper 2 cell cytokine production [GO:0035745] Sources: GOC:obol Definition: Any process that stops, prevents or reduces the frequency, rate or extent of T-helper 2 cell cytokine production.